sensory perception of umami taste [GO:0050917] (biological process) Also known as: umami taste perception Relationships: is a type of sensory perception of taste [GO:0050909] Sources: GOC:ai Definition: The series of events required to receive an umami taste stimulus, convert it to a molecular signal, and recognize and characterize the signal. Umami taste is the savory taste of meats and other foods that are rich in glutamates. This is a neurological process.